{
  "gene_name": "Pre-mRNA-splicing factor ISY1 homolog",
  "gene_symbol": "ISY1",
  "term_label": "Unknown molecular function",
  "gene": "UniProtKB:Q9ULR0",
  "term_id": "UNKNOWN:0001"
}